{
  "gene": "UniProtKB:O43915",
  "term_label": "response to hypoxia",
  "term_id": "GO:0001666",
  "gene_name": "Vascular endothelial growth factor D",
  "gene_symbol": "VEGFD"
}